{
  "gene_symbol": "TMEM218",
  "gene_name": "Transmembrane protein 218",
  "term_label": "Unknown molecular function",
  "gene": "UniProtKB:A2RU14",
  "term_id": "UNKNOWN:0001"
}